{
  "gene": "UniProtKB:Q6ZUX7",
  "term_id": "GO:0016020",
  "term_label": "membrane",
  "gene_name": "LHFPL tetraspan subfamily member 2 protein",
  "gene_symbol": "LHFPL2"
}